{
  "term_id": "GO:0030126",
  "gene": "UniProtKB:Q8NDZ4",
  "term_label": "COPI vesicle coat",
  "gene_name": "Divergent protein kinase domain 2A",
  "gene_symbol": "DIPK2A"
}